{
  "gene_symbol": "ACVRL1",
  "gene": "UniProtKB:P37023",
  "term_label": "SMAD binding",
  "gene_name": "Serine_threonine-protein kinase receptor R3",
  "term_id": "GO:0046332"
}